eukaryotic translation initiation factor 2 complex [GO:0005850] (cellular component) Also known as: eIF-2, eIF2 Definition: Complex of three heterogeneous polypeptide chains, that form a ternary complex with initiator methionyl-tRNA and GTP. This ternary complex binds to free 40S subunit, which subsequently binds the 5' end of mRNA. Relationships: is a type of protein-containing complex [GO:0032991]; is part of cytoplasm [GO:0005737] References: PMID:10216940